{
  "term_label": "cytoplasm",
  "gene_symbol": "EXD2",
  "gene": "UniProtKB:Q9NVH0",
  "gene_name": "Exonuclease 3'-5' domain-containing protein 2",
  "term_id": "GO:0005737"
}